{
  "term_label": "plasma membrane",
  "gene": "UniProtKB:Q99712",
  "gene_symbol": "KCNJ15",
  "term_id": "GO:0005886",
  "gene_name": "ATP-sensitive inward rectifier potassium channel 15"
}